{
  "gene_symbol": "PHC1",
  "term_id": "GO:0042393",
  "term_label": "histone binding",
  "gene": "UniProtKB:P78364",
  "gene_name": "Polyhomeotic-like protein 1"
}